hyphal septin band [GO:0032163] (cellular component) Relationships: is a type of septin band [GO:0032158] References: PMID:16151244 Sources: GOC:krc, GOC:mah Definition: A septin band, i.e. a diffuse ring composed of a series of septin bars running parallel to the long axis of the cell, located at the junction between the mother cell and the germ tube (hypha) of a fungal cell growing filamentously.